{
  "term_id": "GO:0015271",
  "gene_symbol": "KCNK12",
  "term_label": "outward rectifier potassium channel activity",
  "gene": "UniProtKB:Q9HB15",
  "gene_name": "Potassium channel subfamily K member 12"
}